{
  "gene_name": "Paralemmin-3",
  "term_label": "negative regulation of cytokine-mediated signaling pathway",
  "gene_symbol": "PALM3",
  "gene": "UniProtKB:A6NDB9",
  "term_id": "GO:0001960"
}